{
  "term_id": "UNKNOWN:0001",
  "gene_name": "Transmembrane protein 121",
  "term_label": "Unknown molecular function",
  "gene": "UniProtKB:Q9BTD3",
  "gene_symbol": "TMEM121"
}